{
  "gene": "UniProtKB:Q9HAP2",
  "gene_name": "MLX-interacting protein",
  "term_label": "DNA-binding transcription factor activity, RNA polymerase II-specific",
  "gene_symbol": "MLXIP",
  "term_id": "GO:0000981"
}